{
  "term_id": "GO:0010803",
  "term_label": "regulation of tumor necrosis factor-mediated signaling pathway",
  "gene_symbol": "SPATA2",
  "gene_name": "Spermatogenesis-associated protein 2",
  "gene": "UniProtKB:Q9UM82"
}